{
  "term_label": "cytosol",
  "gene": "UniProtKB:Q7Z2W4",
  "term_id": "GO:0005829",
  "gene_symbol": "ZC3HAV1",
  "gene_name": "Zinc finger CCCH-type antiviral protein 1"
}